{
  "gene_name": "G-protein coupled receptor 157",
  "gene": "UniProtKB:Q5UAW9",
  "gene_symbol": "GPR157",
  "term_label": "plasma membrane",
  "term_id": "GO:0005886"
}